{
  "term_id": "GO:0005886",
  "term_label": "plasma membrane",
  "gene_name": "Olfactory receptor 2L5",
  "gene_symbol": "OR2L5",
  "gene": "UniProtKB:Q8NG80"
}